{
  "term_id": "GO:0098839",
  "term_label": "postsynaptic density membrane",
  "gene": "UniProtKB:Q14957",
  "gene_symbol": "GRIN2C",
  "gene_name": "Glutamate receptor ionotropic, NMDA 2C"
}